D-xylose transmembrane transporter activity [GO:0015148] (molecular function) Subtypes: D-xylose:proton symporter activity [GO:0015519], ABC-type D-xylose transporter activity [GO:0015614] Relationships: is a type of pentose transmembrane transporter activity [GO:0015146]; BFO_0000050 D-xylose transmembrane transport [GO:0015753] Sources: GOC:mtg_transport, ISBN:0198506732, ISBN:0815340729 Definition: Enables the transfer of D-xylose from one side of a membrane to the other. D-xylose (the naturally occurring enantiomer is always D-) is a constituent of plant polysaccharides.